{
  "gene_name": "MORF4 family associated protein 1 like 2",
  "term_label": "Unknown cellular component",
  "gene": "UniProtKB:B2RBV5",
  "term_id": "UNKNOWN:0003",
  "gene_symbol": "MRFAP1L2"
}